{
  "gene_symbol": "SGPP1",
  "term_label": "sphingosine metabolic process",
  "gene_name": "Sphingosine-1-phosphate phosphatase 1",
  "term_id": "GO:0006670",
  "gene": "UniProtKB:Q9BX95"
}